{
  "gene": "UniProtKB:A0A286YF18",
  "gene_name": "Small integral membrane protein 44",
  "gene_symbol": "SMIM44",
  "term_id": "UNKNOWN:0003",
  "term_label": "Unknown cellular component"
}